{
  "gene_name": "Glutamine-rich protein 2",
  "gene_symbol": "QRICH2",
  "term_id": "GO:0030317",
  "gene": "UniProtKB:Q9H0J4",
  "term_label": "flagellated sperm motility"
}